aminoglycoside 3-N-acetyltransferase activity [GO:0046353] (molecular function) Sources: RHEA:12665 Also known as: gentamycin 3-N-acetyltransferase activity, acetyl-CoA:gentamicin-C N3-acetyltransferase activity, gentamicin 3-N-acetyltransferase activity, gentamicin acetyltransferase I activity, gentamicin-(3)-N-acetyltransferase activity, 3-N-aminoglycoside acetyltransferase activity, 3-aminoglycoside acetyltransferase activity, acetyl-CoA:2-deoxystreptamine-antibiotic N3-acetyltransferase activity, aminoglycoside acetyltransferase AAC(3)-1, aminoglycoside acetyltransferase AAC(3)-I activity, gentamycin acetyltransferase I Definition: Catalysis of the reaction: a 2-deoxystreptamine antibiotic + acetyl-CoA = an N(3)-acetyl-2-deoxystreptamine antibiotic + CoA + H+. Relationships: is a type of GO:0034069